{
  "gene": "UniProtKB:Q96Q35",
  "gene_symbol": "FLACC1",
  "term_label": "Unknown molecular function",
  "gene_name": "Flagellum-associated coiled-coil domain-containing protein 1",
  "term_id": "UNKNOWN:0001"
}